left/right axis specification [GO:0070986] (biological process) Sources: GOC:dph, GOC:gvg, GOC:mah Also known as: left-right axis specification, left/right axis determination Relationships: is a type of GO:0009798; is part of GO:0060972 Definition: The establishment, maintenance and elaboration of the left/right axis. The left/right axis is defined by a line that runs orthogonal to both the anterior/posterior and dorsal/ventral axes. Each side is defined from the viewpoint of the organism rather of the observer (as per anatomical axes).